{
  "gene_symbol": "TCF25",
  "term_id": "UNKNOWN:0001",
  "gene": "UniProtKB:Q9BQ70",
  "term_label": "Unknown molecular function",
  "gene_name": "Ribosome quality control complex subunit TCF25"
}